{
  "gene": "UniProtKB:Q13569",
  "term_label": "base-excision repair, AP site formation",
  "gene_name": "G_T mismatch-specific thymine DNA glycosylase",
  "term_id": "GO:0006285",
  "gene_symbol": "TDG"
}